{
  "term_id": "GO:0030289",
  "gene_name": "Protein PPP4R3C",
  "gene_symbol": "PPP4R3C",
  "term_label": "protein phosphatase 4 complex",
  "gene": "UniProtKB:Q6ZMV5"
}